positive regulation of intermediate mesodermal cell fate specification [GO:0048400] (biological process) Relationships: is a type of GO:0048337; is a type of regulation of intermediate mesodermal cell fate specification [GO:0048399]; positively regulates intermediate mesodermal cell fate specification [GO:0048398] Also known as: up regulation of intermediate mesodermal cell fate specification, up-regulation of intermediate mesodermal cell fate specification, upregulation of intermediate mesodermal cell fate specification, activation of intermediate mesodermal cell fate specification, stimulation of intermediate mesodermal cell fate specification Sources: GOC:dgh Definition: Any process that activates or increases the frequency, rate or extent of intermediate mesoderm cell fate specification.